{
  "gene": "UniProtKB:Q9H4A5",
  "term_label": "trans-Golgi network",
  "gene_name": "Golgi phosphoprotein 3-like",
  "gene_symbol": "GOLPH3L",
  "term_id": "GO:0005802"
}